{
  "term_id": "GO:0000209",
  "gene_name": "E3 ubiquitin-protein ligase RNF166",
  "gene_symbol": "RNF166",
  "gene": "UniProtKB:Q96A37",
  "term_label": "protein polyubiquitination"
}